{
  "gene_symbol": "CDCA7L",
  "term_label": "nucleus",
  "term_id": "GO:0005634",
  "gene_name": "Cell division cycle-associated 7-like protein",
  "gene": "UniProtKB:Q96GN5"
}